{
  "term_id": "GO:0060070",
  "gene_name": "Segment polarity protein dishevelled homolog DVL-3",
  "gene": "UniProtKB:Q92997",
  "term_label": "canonical Wnt signaling pathway",
  "gene_symbol": "DVL3"
}